{
  "gene_symbol": "RPL34",
  "term_label": "cytosolic large ribosomal subunit",
  "gene_name": "Large ribosomal subunit protein eL34",
  "term_id": "GO:0022625",
  "gene": "UniProtKB:P49207"
}